{
  "gene": "UniProtKB:Q8NH74",
  "gene_name": "Olfactory receptor 10A6",
  "gene_symbol": "OR10A6",
  "term_id": "GO:0004984",
  "term_label": "olfactory receptor activity"
}